response to selenium ion [GO:0010269] (biological process) Definition: Any process that results in a change in state or activity of a cell or an organism (in terms of movement, secretion, enzyme production, gene expression, etc.) as a result of a stimulus from selenium ion. Subtypes: cellular response to selenium ion [GO:0071291] Relationships: is_a response to chemical [GO:0042221] Sources: GOC:mg